{
  "gene_name": "Zinc finger protein 75D",
  "term_label": "Unknown cellular component",
  "term_id": "UNKNOWN:0003",
  "gene": "UniProtKB:P51815",
  "gene_symbol": "ZNF75D"
}